{
  "gene_name": "Eukaryotic initiation factor 4A-I",
  "gene_symbol": "EIF4A1",
  "term_id": "GO:0002183",
  "term_label": "cytoplasmic translational initiation",
  "gene": "UniProtKB:P60842"
}